{
  "term_label": "actin filament binding",
  "gene": "UniProtKB:Q13796",
  "gene_symbol": "SHROOM2",
  "term_id": "GO:0051015",
  "gene_name": "Protein Shroom2"
}